{
  "term_id": "GO:0030488",
  "gene": "UniProtKB:Q9Y2Z2",
  "gene_name": "Protein MTO1 homolog, mitochondrial",
  "gene_symbol": "MTO1",
  "term_label": "tRNA methylation"
}